{
  "gene": "UniProtKB:Q14532",
  "term_id": "GO:0030855",
  "gene_name": "Keratin, type I cuticular Ha2",
  "term_label": "epithelial cell differentiation",
  "gene_symbol": "KRT32"
}